{
  "gene_name": "Protein mono-ADP-ribosyltransferase TIPARP",
  "term_id": "GO:0003950",
  "term_label": "NAD+ poly-ADP-ribosyltransferase activity",
  "gene_symbol": "TIPARP",
  "gene": "UniProtKB:Q7Z3E1"
}